{
  "gene_name": "Ankyrin repeat and SOCS box protein 18",
  "gene": "UniProtKB:Q6ZVZ8",
  "gene_symbol": "ASB18",
  "term_label": "Unknown biological process",
  "term_id": "UNKNOWN:0002"
}